{
  "gene_name": "Phosphomannomutase 2",
  "gene_symbol": "PMM2",
  "term_id": "GO:0006487",
  "term_label": "protein N-linked glycosylation",
  "gene": "UniProtKB:O15305"
}